{
  "gene_name": "Putative protein FAM86C2P",
  "gene_symbol": "FAM86C2P",
  "term_label": "Unknown molecular function",
  "gene": "UniProtKB:A6NEL3",
  "term_id": "UNKNOWN:0001"
}